{
  "gene_symbol": "TIAM2",
  "term_id": "GO:0045202",
  "term_label": "synapse",
  "gene_name": "Rho guanine nucleotide exchange factor TIAM2",
  "gene": "UniProtKB:Q8IVF5"
}